{
  "gene_name": "Sodium_calcium exchanger 2",
  "gene": "UniProtKB:Q9UPR5",
  "gene_symbol": "SLC8A2",
  "term_id": "GO:0005432",
  "term_label": "calcium:sodium antiporter activity"
}